{
  "term_label": "immune response",
  "term_id": "GO:0006955",
  "gene_name": "Low affinity immunoglobulin epsilon Fc receptor",
  "gene_symbol": "FCER2",
  "gene": "UniProtKB:P06734"
}